regulation of immune system process [GO:0002682] (biological process) Subtypes: regulation of antigen processing and presentation [GO:0002577], regulation of tolerance induction [GO:0002643], negative regulation of immune system process [GO:0002683], positive regulation of immune system process [GO:0002684], regulation of leukocyte migration [GO:0002685], GO:0002694, regulation of immune effector process [GO:0002697], GO:0002905, GO:0033025, regulation of neutrophil apoptotic process [GO:0033029], GO:0035206, regulation of hemocyte differentiation [GO:0045610], GO:0050776, regulation of activation-induced cell death of T cells [GO:0070235], regulation of activated T cell autonomous cell death [GO:0070239], GO:1903706 Relationships: is a type of regulation of biological process [GO:0050789]; regulates immune system process [GO:0002376] Sources: GOC:add Definition: Any process that modulates the frequency, rate, or extent of an immune system process.